{
  "gene_symbol": "IL2RG",
  "gene": "UniProtKB:P31785",
  "term_id": "GO:0019221",
  "gene_name": "Cytokine receptor common subunit gamma",
  "term_label": "cytokine-mediated signaling pathway"
}